{
  "term_id": "UNKNOWN:0003",
  "gene": "UniProtKB:P33076",
  "gene_name": "MHC class II transactivator",
  "term_label": "Unknown cellular component",
  "gene_symbol": "CIITA"
}